positive regulation of fever generation by positive regulation of prostaglandin secretion [GO:0071812] (biological process) Definition: Any process that increases the rate or extent of fever generation via positive regulation of the frequency, rate or extent of the regulated release of a prostaglandin from a cell. Sources: GOC:BHF, GOC:dph, GOC:mah Relationships: is_a positive regulation of fever generation [GO:0031622]; is a type of positive regulation of prostaglandin secretion [GO:0032308]